{
  "term_id": "GO:0046961",
  "gene": "UniProtKB:P21283",
  "gene_symbol": "ATP6V1C1",
  "gene_name": "V-type proton ATPase subunit C 1",
  "term_label": "proton-transporting ATPase activity, rotational mechanism"
}